{
  "term_id": "GO:0005811",
  "term_label": "lipid droplet",
  "gene": "UniProtKB:Q8NBQ5",
  "gene_name": "Estradiol 17-beta-dehydrogenase 11",
  "gene_symbol": "HSD17B11"
}